{
  "gene": "UniProtKB:Q9P1A6",
  "gene_name": "Disks large-associated protein 2",
  "term_id": "GO:0050804",
  "term_label": "modulation of chemical synaptic transmission",
  "gene_symbol": "DLGAP2"
}